{
  "gene_symbol": "SLC25A41",
  "gene": "UniProtKB:Q8N5S1",
  "term_id": "GO:0015866",
  "term_label": "ADP transport",
  "gene_name": "Mitochondrial carrier protein SCaMC-3L"
}